{
  "gene": "UniProtKB:Q9NPI9",
  "term_label": "potassium ion import across plasma membrane",
  "gene_name": "Inward rectifier potassium channel 16",
  "term_id": "GO:1990573",
  "gene_symbol": "KCNJ16"
}